{
  "gene_name": "Olfactory receptor 51Q1",
  "gene_symbol": "OR51Q1",
  "term_label": "olfactory receptor activity",
  "term_id": "GO:0004984",
  "gene": "UniProtKB:Q8NH59"
}